protein-N(PI)-phosphohistidine-galactosamine phosphotransferase system transporter activity [GO:0022876] (MF) Definition: Catalysis of the PEP-dependent, phosphoryl transfer-driven transport of substances across a membrane. The transport happens by catalysis of the reaction: protein N-phosphohistidine + galactosamine(out) = protein histidine + galactosamine phosphate(in). This differs from primary and secondary active transport in that the solute is modified during transport. Also known as: galactosamine PTS transporter activity Sources: GOC:mtg_transport, ISBN:0815340729 Relationships: is a type of protein-N(PI)-phosphohistidine-sugar phosphotransferase activity [GO:0008982]; is a type of GO:0019196